{
  "term_id": "GO:0003993",
  "gene_symbol": "ACP2",
  "gene": "UniProtKB:P11117",
  "term_label": "acid phosphatase activity",
  "gene_name": "Lysosomal acid phosphatase"
}